{
  "gene": "UniProtKB:Q8MH63",
  "gene_symbol": "SLC7A5P1",
  "gene_name": "Putative L-type amino acid transporter 1-like protein MLAS",
  "term_label": "Unknown biological process",
  "term_id": "UNKNOWN:0002"
}